{
  "gene": "UniProtKB:Q5MNZ6",
  "term_label": "autophagy of mitochondrion",
  "gene_symbol": "WDR45B",
  "gene_name": "WD repeat domain phosphoinositide-interacting protein 3",
  "term_id": "GO:0000422"
}